{
  "term_label": "cytoplasm",
  "term_id": "GO:0005737",
  "gene": "UniProtKB:Q6P597",
  "gene_symbol": "KLC3",
  "gene_name": "Kinesin light chain 3"
}